{
  "gene_name": "Disintegrin and metalloproteinase domain-containing protein 20",
  "term_label": "male gonad development",
  "term_id": "GO:0008584",
  "gene_symbol": "ADAM20",
  "gene": "UniProtKB:O43506"
}